{
  "term_label": "signaling receptor binding",
  "gene_name": "Tyrosine-protein kinase Blk",
  "term_id": "GO:0005102",
  "gene": "UniProtKB:P51451",
  "gene_symbol": "BLK"
}